{
  "gene": "UniProtKB:Q9UJX6",
  "term_id": "GO:0007091",
  "gene_name": "Anaphase-promoting complex subunit 2",
  "term_label": "metaphase/anaphase transition of mitotic cell cycle",
  "gene_symbol": "ANAPC2"
}